{
  "gene_symbol": "METTL8",
  "term_id": "UNKNOWN:0002",
  "gene": "UniProtKB:Q9H825",
  "gene_name": "tRNA N(3)-methylcytidine methyltransferase METTL8, mitochondrial",
  "term_label": "Unknown biological process"
}